{
  "term_id": "UNKNOWN:0001",
  "term_label": "Unknown molecular function",
  "gene_name": "Putative ubiquitin-conjugating enzyme E2 D2-like protein",
  "gene": "UniProtKB:Q8IWF7",
  "gene_symbol": "UBE2DNL"
}